{
  "term_id": "GO:0060385",
  "gene_symbol": "NPTX1",
  "gene": "UniProtKB:Q15818",
  "gene_name": "Neuronal pentraxin-1",
  "term_label": "axonogenesis involved in innervation"
}